{
  "gene_symbol": "EXOSC5",
  "term_id": "GO:0005730",
  "gene": "UniProtKB:Q9NQT4",
  "gene_name": "Exosome complex component RRP46",
  "term_label": "nucleolus"
}